uncoating of virus [GO:0019061] (biological process) References: PMID:8162442 Sources: GOC:plm, ISBN:0781702534 Definition: The process by which an incoming virus is disassembled in the host cell to release a replication-competent viral genome. Relationships: is a type of viral process [GO:0016032] Also known as: viral uncoating